{
  "gene_name": "Keratin, type II cytoskeletal 73",
  "gene": "UniProtKB:Q86Y46",
  "term_id": "GO:0031424",
  "gene_symbol": "KRT73",
  "term_label": "keratinization"
}